{
  "gene_name": "snRNA-activating protein complex subunit 4",
  "gene": "UniProtKB:Q5SXM2",
  "term_label": "snRNA transcription by RNA polymerase III",
  "term_id": "GO:0042796",
  "gene_symbol": "SNAPC4"
}